{
  "term_label": "lipoprotein lipase activity",
  "gene_name": "Endothelial lipase",
  "gene_symbol": "LIPG",
  "term_id": "GO:0004465",
  "gene": "UniProtKB:Q9Y5X9"
}